negative regulation of protein O-linked glycosylation [GO:1904099] (biological process) Definition: Any process that stops, prevents or reduces the frequency, rate or extent of protein O-linked glycosylation. Relationships: is a type of GO:0010561; is a type of regulation of protein O-linked glycosylation [GO:1904098]; negatively regulates protein O-linked glycosylation [GO:0006493] Also known as: down regulation of protein O-linked glycosylation, down regulation of protein amino acid O-linked glycosylation, down-regulation of protein O-linked glycosylation, down-regulation of protein amino acid O-linked glycosylation, downregulation of protein O-linked glycosylation, downregulation of protein amino acid O-linked glycosylation, negative regulation of protein amino acid O-linked glycosylation, inhibition of protein O-linked glycosylation, inhibition of protein amino acid O-linked glycosylation References: PMID:24509081 Sources: GOC:TermGenie, GO_REF:0000058